misfolded protein binding [GO:0051787] (molecular function) Definition: Binding to a misfolded protein. Sources: GOC:ai Relationships: is a type of protein binding [GO:0005515]